host-mediated modulation of oral microbiota composition [GO:0120332] (biological process) Also known as: host-mediated regulation of oral microbiota composition, host-induced regulation of oral microbiota composition References: PMID:31882545 Relationships: is a type of homeostasis of number of cells [GO:0048872]; is a type of host-mediated perturbation of symbiont process [GO:0051851] Definition: The biological process involved in maintaining the steady-state number of cells within a population of free-living cells, such as the bacteria, in the mouth.